{
  "term_label": "Unknown cellular component",
  "gene_name": "Transmembrane protein 53",
  "gene_symbol": "TMEM53",
  "term_id": "UNKNOWN:0003",
  "gene": "UniProtKB:Q6P2H8"
}